dimethyl sulfide monooxygenase activity [GO:0018633] (molecular function) Relationships: is a type of oxidoreductase activity, acting on paired donors, with incorporation or reduction of molecular oxygen, NAD(P)H as one donor, and incorporation of one atom of oxygen [GO:0016709] Also known as: dimethyl sulphide monooxygenase activity Definition: Catalysis of the reaction: dimethyl sulfide + H+ + NADH + O2 = formaldehyde + H2O + methanethiol + NAD+. References: PMID:21216999 Sources: RHEA:31355